hydroxylamine reductase activity [GO:0050418] (molecular function) Sources: EC:1.7.99.1 Definition: Catalysis of the reaction: NH3 + H2O + acceptor = hydroxylamine + reduced acceptor. Also known as: ammonia:(acceptor) oxidoreductase activity, ammonia:acceptor oxidoreductase activity, hydroxylamine (acceptor) reductase activity Relationships: is a type of oxidoreductase activity, acting on other nitrogenous compounds as donors [GO:0016661]